{
  "gene_symbol": "TRAPPC2B",
  "term_id": "GO:0030008",
  "term_label": "TRAPP complex",
  "gene_name": "Trafficking protein particle complex subunit 2B",
  "gene": "UniProtKB:P0DI82"
}